{
  "gene": "UniProtKB:Q6IPU0",
  "gene_symbol": "CENPP",
  "term_label": "Unknown biological process",
  "gene_name": "Centromere protein P",
  "term_id": "UNKNOWN:0002"
}